{
  "term_label": "protein O-linked glycosylation via mannose",
  "gene_symbol": "RXYLT1",
  "gene": "UniProtKB:Q9Y2B1",
  "gene_name": "Ribitol-5-phosphate xylosyltransferase 1",
  "term_id": "GO:0035269"
}